{
  "gene_symbol": "STMN2",
  "gene_name": "Stathmin-2",
  "term_id": "GO:0031175",
  "term_label": "neuron projection development",
  "gene": "UniProtKB:Q93045"
}